{
  "gene_symbol": "MEN1",
  "gene_name": "Menin",
  "term_id": "GO:0045786",
  "gene": "UniProtKB:O00255",
  "term_label": "negative regulation of cell cycle"
}